negative regulation of endosperm development [GO:1904095] (biological process) Relationships: is a type of GO:0051093; is a type of regulation of endosperm development [GO:2000014]; is a type of GO:2000242; negatively regulates endosperm development [GO:0009960] Definition: Any process that stops, prevents or reduces the frequency, rate or extent of endosperm development. Also known as: down regulation of endosperm development, down-regulation of endosperm development, downregulation of endosperm development, inhibition of endosperm development References: PMID:25194028 Sources: GOC:TermGenie, GO_REF:0000058